{
  "gene_name": "Protein LDOC1",
  "term_id": "UNKNOWN:0001",
  "gene": "UniProtKB:O95751",
  "gene_symbol": "LDOC1",
  "term_label": "Unknown molecular function"
}